phototransduction [GO:0007602] (biological process) Also known as: phototransduction, visible light, light adaptation, phototrophin mediated phototransduction, opsin Definition: The sequence of reactions within a cell required to convert absorbed photons into a molecular signal. Sources: GOC:go_curators Relationships: is a type of GO:0007165; is_a detection of light stimulus [GO:0009583] Subtypes: phototransduction, visible light [GO:0007603], phototransduction, UV [GO:0007604], red, far-red light phototransduction [GO:0009585], UV-A, blue light phototransduction [GO:0009588], GO:0016056